cellular response to leptomycin B [GO:0072750] (biological process) Sources: GOC:mah Definition: Any process that results in a change in state or activity of a cell (in terms of movement, secretion, enzyme production, gene expression, etc.) as a result of a leptomycin B stimulus. Relationships: is a type of GO:0071398; is a type of response to leptomycin B [GO:1901344]